apicomedial cortex [GO:0106037] (cellular component) Definition: The region that lies just beneath the plasma membrane in the middle of the apical edge of a cell. Also known as: medioapical cortex Relationships: is a type of apical cortex [GO:0045179]; is part of apical cortex [GO:0045179] References: PMID:23831726, PMID:28263180